response to spindle checkpoint signaling [GO:0072417] (biological process) Subtypes: GO:0072476, response to spindle assembly checkpoint signaling [GO:0072485] Also known as: response to signal involved in spindle checkpoint, spindle checkpoint effector process Definition: A process that occurs in response to signals generated as a result of spindle checkpoint signaling. Sources: GOC:mtg_cell_cycle Relationships: is a type of GO:0072396